negative regulation of extracellular matrix constituent secretion [GO:0003332] (biological process) Definition: Any process that decreases the rate, frequency, or extent the controlled release of molecules that form the extracellular matrix, including carbohydrates and glycoproteins by a cell or a group of cells. Relationships: is a type of regulation of extracellular matrix constituent secretion [GO:0003330]; is a type of negative regulation of extracellular matrix organization [GO:1903054]; is a type of negative regulation of secretion by cell [GO:1903531]; negatively regulates extracellular matrix constituent secretion [GO:0070278] Sources: GOC:dph, GOC:tb